{
  "gene_symbol": "UAP1",
  "term_id": "UNKNOWN:0003",
  "term_label": "Unknown cellular component",
  "gene_name": "UDP-N-acetylhexosamine pyrophosphorylase",
  "gene": "UniProtKB:Q16222"
}